{
  "gene_symbol": "LINS1",
  "term_id": "UNKNOWN:0002",
  "gene": "UniProtKB:Q8NG48",
  "term_label": "Unknown biological process",
  "gene_name": "Protein Lines homolog 1"
}